D-glucose:sodium symporter activity [GO:0005412] (molecular function) Relationships: is a type of carbohydrate:monoatomic cation symporter activity [GO:0005402]; is a type of solute:sodium symporter activity [GO:0015370]; is a type of D-glucose transmembrane transporter activity [GO:0055056] Subtypes: low-affinity D-glucose:sodium symporter activity [GO:0005362] Sources: TC:2.A.21.3.- Definition: Enables the transfer of a solute or solutes from one side of a membrane to the other according to the reaction: D-glucose(out) + Na+(out) = D-glucose(in) + Na+(in). Also known as: glucose:sodium symporter activity, sodium/glucose symporter activity